{
  "term_label": "cilium movement involved in cell motility",
  "gene_symbol": "TEKT5",
  "gene": "UniProtKB:Q96M29",
  "term_id": "GO:0060294",
  "gene_name": "Tektin-5"
}